{
  "term_id": "GO:0010508",
  "gene": "UniProtKB:P19484",
  "gene_symbol": "TFEB",
  "gene_name": "Transcription factor EB",
  "term_label": "positive regulation of autophagy"
}